{
  "gene": "UniProtKB:Q9H1D9",
  "gene_name": "DNA-directed RNA polymerase III subunit RPC6",
  "term_label": "Unknown biological process",
  "gene_symbol": "POLR3F",
  "term_id": "UNKNOWN:0002"
}